{
  "term_label": "single-stranded DNA binding",
  "gene_name": "DNA helicase MCM8",
  "term_id": "GO:0003697",
  "gene": "UniProtKB:Q9UJA3",
  "gene_symbol": "MCM8"
}